{
  "gene_name": "A disintegrin and metalloproteinase with thrombospondin motifs 14",
  "gene": "UniProtKB:Q8WXS8",
  "term_id": "GO:0006508",
  "gene_symbol": "ADAMTS14",
  "term_label": "proteolysis"
}